{
  "gene": "UniProtKB:Q15853",
  "term_label": "DNA-binding transcription factor activity, RNA polymerase II-specific",
  "term_id": "GO:0000981",
  "gene_name": "Upstream stimulatory factor 2",
  "gene_symbol": "USF2"
}